{
  "term_label": "prostaglandin metabolic process",
  "gene_name": "Aldo-keto reductase family 1 member C3",
  "gene_symbol": "AKR1C3",
  "term_id": "GO:0006693",
  "gene": "UniProtKB:P42330"
}